{
  "gene_symbol": "OR8G1",
  "term_label": "olfactory receptor activity",
  "term_id": "GO:0004984",
  "gene": "UniProtKB:Q15617",
  "gene_name": "Olfactory receptor 8G1"
}